{
  "gene_name": "Zinc finger protein 506",
  "gene": "UniProtKB:Q5JVG8",
  "gene_symbol": "ZNF506",
  "term_label": "regulation of DNA-templated transcription",
  "term_id": "GO:0006355"
}